{
  "term_id": "UNKNOWN:0003",
  "term_label": "Unknown cellular component",
  "gene_symbol": "AGAP7P",
  "gene_name": "Putative Arf-GAP with GTPase, ANK repeat and PH domain-containing protein 7",
  "gene": "UniProtKB:Q5VUJ5"
}